{
  "gene_symbol": "PFKFB3",
  "term_label": "cytosol",
  "gene_name": "6-phosphofructo-2-kinase_fructose-2,6-bisphosphatase 3",
  "gene": "UniProtKB:Q16875",
  "term_id": "GO:0005829"
}